L-lysine 6-transaminase activity [GO:0045484] (molecular function) Relationships: is a type of transaminase activity [GO:0008483] Sources: EC:2.6.1.36, RHEA:21200 Also known as: lysine 6-aminotransferase activity, L-lysine aminotransferase activity, L-lysine transaminase activity, L-lysine-alpha-ketoglutarate 6-aminotransferase activity, L-lysine-alpha-ketoglutarate aminotransferase activity, L-lysine:2-oxoglutarate 6-aminotransferase activity, lysine epsilon-aminotransferase activity, lysine epsilon-transaminase activity, lysine:2-ketoglutarate 6-aminotransferase activity Definition: Catalysis of the reaction: 2-oxoglutarate + L-lysine = L-glutamate + allysine.